{
  "gene_name": "Zinc finger protein 843",
  "gene_symbol": "ZNF843",
  "term_id": "UNKNOWN:0002",
  "gene": "UniProtKB:Q8N446",
  "term_label": "Unknown biological process"
}